{
  "term_label": "Unknown cellular component",
  "gene_name": "RING finger protein 112",
  "gene_symbol": "RNF112",
  "term_id": "UNKNOWN:0003",
  "gene": "UniProtKB:Q9ULX5"
}